regulation of chemokine (C-X-C motif) ligand 2 production [GO:2000341] (biological process) Sources: GOC:BHF, GOC:mah Also known as: regulation of CXCL2 production, regulation of MIP-2 production, regulation of MIP2 production, regulation of SCYB2 production, chemokine (C-C motif) ligand 2 secretion, regulation of CCL2 secretion, regulation of chemokine (C-C motif) ligand 2 secretion Subtypes: negative regulation of chemokine (C-X-C motif) ligand 2 production [GO:2000342], positive regulation of chemokine (C-X-C motif) ligand 2 production [GO:2000343] Definition: Any process that modulates the frequency, rate or extent of chemokine (C-X-C motif) ligand 2 production. Relationships: is a type of regulation of chemokine production [GO:0032642]; regulates chemokine (C-X-C motif) ligand 2 production [GO:0072567]